{
  "gene_name": "Neurogenin-1",
  "gene_symbol": "NEUROG1",
  "term_id": "GO:0007423",
  "term_label": "sensory organ development",
  "gene": "UniProtKB:Q92886"
}